glucagon family peptide binding [GO:0120022] (molecular function) Relationships: is a type of peptide hormone binding [GO:0017046] References: PMID:17715056 Definition: Binding to a member of the glucagon family peptide hormone (e.g. glucagon, glucagon-like peptides, oxyntomodulin, glicentin, ADCYAP1, GHRH, secretin, VIP, GIP). Also known as: glucagon binding, glucagon-like peptide binding